peptidyl-cysteine S-trans-nitrosylation [GO:0035606] (BP) Also known as: protein-to-protein transnitrosylation, S-transnitrosylation, cysteine to cysteine nitrosylation, cysteine-to-cysteine transnitrosylation References: PMID:19854201, PMID:20972425, PMID:20972426 Definition: Transfer of a nitric oxide (NO) group from one cysteine residue to another. Relationships: is a type of GO:0018119